{
  "gene_symbol": "GOLGA5",
  "term_label": "Golgi organization",
  "gene_name": "Golgin subfamily A member 5",
  "term_id": "GO:0007030",
  "gene": "UniProtKB:Q8TBA6"
}